{
  "gene_name": "Factor in the germline alpha",
  "gene": "UniProtKB:Q6QHK4",
  "gene_symbol": "FIGLA",
  "term_id": "GO:0032502",
  "term_label": "developmental process"
}